{
  "term_label": "plasma membrane",
  "term_id": "GO:0005886",
  "gene_symbol": "TMEM119",
  "gene_name": "Transmembrane protein 119",
  "gene": "UniProtKB:Q4V9L6"
}